acyl-lipid (11-3)-desaturase activity [GO:0102003] (molecular function) Relationships: is a type of oxidoreductase activity, acting on paired donors, with oxidation of a pair of donors resulting in the reduction of molecular oxygen to two molecules of water [GO:0016717] Definition: Catalysis of the reaction: an (11Z,14Z)-icosadienoyl-containing glycerolipid + 2 Fe(II)-[cytochrome b5] + 2 H+ + O2 = an (8Z,11Z,14Z)-icosatrienoyl-containing glycerolipid + 2 Fe(III)-[cytochrome b5] + 2 H2O or an (11Z,14Z,17Z)-icosatrienoyl-containing glycerolipid + 2 Fe(II)-[cytochrome b5] + 2 H+ + O2 = an (8Z,11Z,14Z,17Z)-eicosatetraenoyl-containing glycerolipid + 2 Fe(III)-[cytochrome b5] + 2 H2O. Sources: EC:1.14.19.4 Also known as: Delta(8)-desaturase, Delta8-sphingolipid desaturase activity, acyl-lipid 8-desaturase